{
  "gene_name": "Zinc finger protein 3",
  "gene": "UniProtKB:P17036",
  "term_id": "GO:0000981",
  "gene_symbol": "ZNF3",
  "term_label": "DNA-binding transcription factor activity, RNA polymerase II-specific"
}